{
  "gene_name": "Heme transporter HRG1",
  "term_label": "heme binding",
  "gene_symbol": "SLC48A1",
  "gene": "UniProtKB:Q6P1K1",
  "term_id": "GO:0020037"
}